{
  "gene_symbol": "PAFAH1B1",
  "term_label": "nuclear migration",
  "gene_name": "Platelet-activating factor acetylhydrolase IB subunit beta",
  "gene": "UniProtKB:P43034",
  "term_id": "GO:0007097"
}